{
  "gene_symbol": "IQCN",
  "gene": "UniProtKB:Q9H0B3",
  "gene_name": "IQ domain-containing protein N",
  "term_id": "UNKNOWN:0002",
  "term_label": "Unknown biological process"
}